{
  "term_id": "GO:0000226",
  "gene_name": "Microtubule-associated protein 2",
  "term_label": "microtubule cytoskeleton organization",
  "gene_symbol": "MAP2",
  "gene": "UniProtKB:P11137"
}